regulation of interleukin-35-mediated signaling pathway [GO:0070758] (biological process) Sources: GOC:mah Subtypes: GO:0070759, positive regulation of interleukin-35-mediated signaling pathway [GO:0070760] Definition: Any process that modulates the rate, frequency or extent of an interleukin-35-mediated signaling pathway. Relationships: is a type of GO:0001959; regulates interleukin-35-mediated signaling pathway [GO:0070757] Also known as: regulation of IL-35-mediated signaling pathway, regulation of interleukin-35-mediated signalling pathway